{
  "term_label": "Unknown biological process",
  "gene": "UniProtKB:Q8IUK5",
  "term_id": "UNKNOWN:0002",
  "gene_symbol": "PLXDC1",
  "gene_name": "Plexin domain-containing protein 1"
}